{
  "term_id": "GO:0032436",
  "gene_name": "PABIR family member 1",
  "term_label": "positive regulation of proteasomal ubiquitin-dependent protein catabolic process",
  "gene_symbol": "PABIR3",
  "gene": "UniProtKB:Q6P4D5"
}